{
  "gene_symbol": "FER",
  "term_id": "GO:0038095",
  "gene_name": "Tyrosine-protein kinase Fer",
  "term_label": "Fc-epsilon receptor signaling pathway",
  "gene": "UniProtKB:P16591"
}